mitomycin C biosynthetic process [GO:1901777] (biological process) Definition: The chemical reactions and pathways resulting in the formation of mitomycin C. Relationships: is_a ketone biosynthetic process [GO:0042181] Also known as: mitomycin C anabolism, mitomycin C biosynthesis, mitomycin C formation, mitomycin C synthesis References: PMID:10094699, PMID:10099135 Sources: GOC:TermGenie, GOC:yaf, UniPathway:UPA00851